cardioblast cell fate commitment [GO:0042684] (biological process) Sources: GOC:go_curators Definition: The process in which a cell becomes committed to becoming a cardioblast. A cardioblast is a cardiac precursor cell. It is a cell that has been committed to a cardiac fate, but will undergo more cell division rather than terminally differentiating. Relationships: is a type of cardiac cell fate commitment [GO:0060911]; is part of cardioblast differentiation [GO:0010002]